violaceol II biosynthetic process [GO:1900593] (BP) Definition: The chemical reactions and pathways resulting in the formation of violaceol II. Relationships: is a type of GO:0009713; is a type of secondary metabolite biosynthetic process [GO:0044550]; is a type of violaceol II metabolic process [GO:1900591]; is a type of GO:1901503 Also known as: violaceol II anabolism, violaceol II biosynthesis, violaceol II formation, violaceol II synthesis Regulation: RO_0002211 by GO:1900716; negatively regulated by GO:1900717; positively regulated by positive regulation of violaceol II biosynthetic process [GO:1900718] Sources: GOC:TermGenie, GOC:di